{
  "gene_symbol": "BCAR1",
  "term_label": "cell surface receptor protein tyrosine kinase signaling pathway",
  "gene": "UniProtKB:P56945",
  "term_id": "GO:0007169",
  "gene_name": "Breast cancer anti-estrogen resistance protein 1"
}